formate dehydrogenase (NADP+) activity [GO:0047899] (MF) Definition: Catalysis of the reaction: formate + NADP+ = CO2 + NADPH. Sources: EC:1.17.1.10, RHEA:12000 Also known as: NADP-dependent formate dehydrogenase activity, formate:NADP+ oxidoreductase activity Relationships: is a type of oxidoreductase activity, acting on the aldehyde or oxo group of donors, NAD or NADP as acceptor [GO:0016620]